D-serine biosynthetic process [GO:0070179] (biological process) Relationships: is a type of D-amino acid biosynthetic process [GO:0046437]; is a type of GO:0070178 Also known as: D-serine anabolism, D-serine biosynthesis, D-serine formation, D-serine synthesis Sources: CHEBI:16523, GOC:jsg, GOC:mah Definition: The chemical reactions and pathways resulting in the formation of D-serine, the D-enantiomer of serine, i.e. (2R)-2-amino-3-hydroxypropanoic acid. D-serine is often formed by racemization of L-serine.